{
  "gene_name": "HEAT repeat-containing protein 5A",
  "term_label": "retrograde transport, endosome to Golgi",
  "gene_symbol": "HEATR5A",
  "gene": "UniProtKB:Q86XA9",
  "term_id": "GO:0042147"
}